{
  "term_id": "GO:0006457",
  "gene_name": "T-complex protein 1 subunit zeta-2",
  "gene_symbol": "CCT6B",
  "gene": "UniProtKB:Q92526",
  "term_label": "protein folding"
}